{
  "term_id": "GO:0005457",
  "term_label": "GDP-fucose transmembrane transporter activity",
  "gene": "UniProtKB:Q96A29",
  "gene_name": "GDP-fucose transporter 1",
  "gene_symbol": "SLC35C1"
}